{
  "term_id": "GO:0045595",
  "term_label": "regulation of cell differentiation",
  "gene_name": "Runt-related transcription factor 3",
  "gene_symbol": "RUNX3",
  "gene": "UniProtKB:Q13761"
}